{
  "gene": "UniProtKB:Q01433",
  "gene_symbol": "AMPD2",
  "term_id": "GO:0006188",
  "gene_name": "AMP deaminase 2",
  "term_label": "IMP biosynthetic process"
}